{
  "gene_symbol": "ZNRF2",
  "term_label": "ubiquitin protein ligase activity",
  "gene_name": "E3 ubiquitin-protein ligase ZNRF2",
  "term_id": "GO:0061630",
  "gene": "UniProtKB:Q8NHG8"
}